serine transport [GO:0032329] (BP) Also known as: serine import Relationships: is a type of organic cation transport [GO:0015695]; is a type of neutral amino acid transport [GO:0015804]; is a type of GO:0046942; is_a nitrogen compound transport [GO:0071705] Sources: GOC:mah Subtypes: GO:0015825, D-serine transmembrane transport [GO:0042942], serine import across plasma membrane [GO:0098718], serine import into mitochondrion [GO:0140300] Definition: The directed movement of L-serine, 2-amino-3-hydroxypropanoic acid, into, out of or within a cell, or between cells, by means of some agent such as a transporter or pore.